{
  "term_label": "modification-dependent protein catabolic process",
  "gene_name": "Ubiquitin-ribosomal protein eL40 fusion protein",
  "term_id": "GO:0019941",
  "gene": "UniProtKB:P62987",
  "gene_symbol": "UBA52"
}